{
  "term_id": "GO:0008273",
  "gene_name": "Sodium_potassium_calcium exchanger 5",
  "gene_symbol": "SLC24A5",
  "term_label": "calcium, potassium:sodium antiporter activity",
  "gene": "UniProtKB:Q71RS6"
}